{
  "term_label": "plasma membrane",
  "gene_symbol": "GPR83",
  "term_id": "GO:0005886",
  "gene": "UniProtKB:Q9NYM4",
  "gene_name": "G-protein coupled receptor 83"
}